{
  "term_id": "GO:0002476",
  "term_label": "antigen processing and presentation of endogenous peptide antigen via MHC class Ib",
  "gene_symbol": "HLA-F",
  "gene": "UniProtKB:P30511",
  "gene_name": "HLA class I histocompatibility antigen, alpha chain F"
}